{
  "term_id": "GO:0036126",
  "term_label": "sperm flagellum",
  "gene_name": "Dynein regulatory complex protein 9",
  "gene_symbol": "IQCG",
  "gene": "UniProtKB:Q9H095"
}